{
  "gene_symbol": "AP5S1",
  "gene_name": "AP-5 complex subunit sigma-1",
  "term_label": "lysosome",
  "term_id": "GO:0005764",
  "gene": "UniProtKB:Q9NUS5"
}